negative regulation of isoprene biosynthetic process [GO:1900948] (biological process) Also known as: down regulation of 2-methyl-1,3-butadiene biosynthesis, down regulation of 2-methyl-1,3-butadiene biosynthetic process, down regulation of hemiterpene biosynthesis, down regulation of hemiterpene biosynthetic process, down regulation of isoprene biosynthetic process, down-regulation of 2-methyl-1,3-butadiene biosynthesis, down-regulation of 2-methyl-1,3-butadiene biosynthetic process, down-regulation of hemiterpene biosynthesis, down-regulation of hemiterpene biosynthetic process, down-regulation of isoprene biosynthetic process, downregulation of 2-methyl-1,3-butadiene biosynthesis, downregulation of 2-methyl-1,3-butadiene biosynthetic process, downregulation of hemiterpene biosynthesis, downregulation of hemiterpene biosynthetic process, downregulation of isoprene biosynthetic process, negative regulation of 2-methyl-1,3-butadiene biosynthesis, negative regulation of 2-methyl-1,3-butadiene biosynthetic process, negative regulation of hemiterpene biosynthesis, negative regulation of hemiterpene biosynthetic process, inhibition of 2-methyl-1,3-butadiene biosynthesis, inhibition of 2-methyl-1,3-butadiene biosynthetic process, inhibition of hemiterpene biosynthesis, inhibition of hemiterpene biosynthetic process, inhibition of isoprene biosynthetic process Relationships: is a type of negative regulation of isoprenoid metabolic process [GO:0045827]; is a type of GO:0051055; is a type of GO:1900912; is a type of regulation of isoprene biosynthetic process [GO:1900947]; negatively regulates isoprene biosynthetic process [GO:0043612] Sources: GOC:TermGenie, GOC:mengo_curators Definition: Any process that stops, prevents or reduces the frequency, rate or extent of isoprene biosynthetic process.